{
  "term_label": "signal transduction",
  "term_id": "GO:0007165",
  "gene": "UniProtKB:Q04917",
  "gene_symbol": "YWHAH",
  "gene_name": "14-3-3 protein eta"
}